{
  "gene_name": "Small ribosomal subunit protein bS16m",
  "gene": "UniProtKB:Q9Y3D3",
  "term_label": "Unknown biological process",
  "gene_symbol": "MRPS16",
  "term_id": "UNKNOWN:0002"
}